{
  "gene": "UniProtKB:O14522",
  "term_label": "neuron projection development",
  "gene_name": "Receptor-type tyrosine-protein phosphatase T",
  "gene_symbol": "PTPRT",
  "term_id": "GO:0031175"
}